{
  "term_label": "negative regulation of toll-like receptor signaling pathway",
  "term_id": "GO:0034122",
  "gene": "UniProtKB:Q9NPR9",
  "gene_symbol": "GPR108",
  "gene_name": "Protein GPR108"
}